sterol sensor activity [GO:0032935] (MF) Also known as: sterol sensing activity, sterol-sensing domain Definition: Binding to and responding, e.g. by conformational change, to changes in the cellular level of a sterol. Relationships: is a type of lipid sensor activity [GO:0106254]; has part sterol binding [GO:0032934] Sources: GOC:mah